{
  "term_label": "immunoglobulin mediated immune response",
  "term_id": "GO:0016064",
  "gene": "UniProtKB:A0A0A0MS14",
  "gene_symbol": "IGHV1-45",
  "gene_name": "Immunoglobulin heavy variable 1-45"
}